{
  "gene_name": "Granzyme M",
  "gene_symbol": "GZMM",
  "term_id": "GO:0005615",
  "term_label": "extracellular space",
  "gene": "UniProtKB:P51124"
}